{
  "term_label": "cytoplasm",
  "gene": "UniProtKB:Q05932",
  "gene_name": "Folylpolyglutamate synthase, mitochondrial",
  "term_id": "GO:0005737",
  "gene_symbol": "FPGS"
}